{
  "gene": "UniProtKB:P55072",
  "gene_name": "Transitional endoplasmic reticulum ATPase",
  "term_id": "GO:0005829",
  "term_label": "cytosol",
  "gene_symbol": "VCP"
}